{
  "term_label": "GTPase activator activity",
  "gene_name": "Guanine nucleotide-binding protein G(q) subunit alpha",
  "gene_symbol": "GNAQ",
  "term_id": "GO:0005096",
  "gene": "UniProtKB:P50148"
}